{
  "gene_symbol": "NFATC3",
  "term_id": "GO:0045944",
  "gene": "UniProtKB:Q12968",
  "gene_name": "Nuclear factor of activated T-cells, cytoplasmic 3",
  "term_label": "positive regulation of transcription by RNA polymerase II"
}